{
  "term_id": "GO:0097190",
  "gene_symbol": "TFPT",
  "gene_name": "TCF3 fusion partner",
  "term_label": "apoptotic signaling pathway",
  "gene": "UniProtKB:P0C1Z6"
}